{
  "term_id": "UNKNOWN:0003",
  "term_label": "Unknown cellular component",
  "gene_symbol": "CD302",
  "gene": "UniProtKB:Q8IX05",
  "gene_name": "CD302 antigen"
}